haltere disc morphogenesis [GO:0007481] (biological process) Definition: The process in which the anatomical structures derived from the haltere disc are generated and organized. This includes the transformation of a haltere imaginal disc from a monolayered epithelium in the larvae of holometabolous insects into the recognizable adult capitellum, pedicel, haltere sclerite, metathoracic spiracle and metanotum. Also known as: haltere disc metamorphosis Relationships: is a type of imaginal disc morphogenesis [GO:0007560]; is part of haltere disc development [GO:0035216] Sources: GOC:bf, ISBN:0879694238